arbuscular mycorrhizal association [GO:0036377] (biological process) Also known as: arbuscular mycorrhizae formation, arbuscular mycorrhizas formation, arbuscular mycorrhizal symbiosis Sources: GOC:sk, Wikipedia:Arbuscular_mycorrhiza Relationships: is a type of biological process involved in symbiotic interaction [GO:0044403] Definition: A form of mutualism between a fungus and the roots of a vascular plant, where hyphae of the fungus penetrate the plant cell wall and invaginate its cell membrane. Once inside, the fungus forms highly branched structures for nutrient exchange with the plant called arbuscules. Aids in the acquisition by the plant of nutrients such as phosphorus from the soil.